{
  "gene_name": "Putative uncharacterized protein PRO0255",
  "term_label": "Unknown molecular function",
  "gene_symbol": "PRO0255",
  "term_id": "UNKNOWN:0001",
  "gene": "UniProtKB:Q9UI72"
}